transferrin receptor binding [GO:1990459] (molecular function) References: PMID:9819414 Sources: GOC:pm Definition: Binding to a transferrin receptor. Relationships: is a type of GO:0005102